{
  "term_id": "UNKNOWN:0001",
  "term_label": "Unknown molecular function",
  "gene_symbol": "SELENOS",
  "gene": "UniProtKB:Q9BQE4",
  "gene_name": "Selenoprotein S"
}